{
  "gene_name": "Unconventional myosin-Ig",
  "gene_symbol": "MYO1G",
  "term_id": "GO:0005902",
  "gene": "UniProtKB:B0I1T2",
  "term_label": "microvillus"
}